EDS1 disease-resistance complex [GO:0106093] (cellular component) Relationships: is a type of GO:0032991 Note: Interacts with the R genes triggering ETI and systemic resistance. Definition: A plant complex involved in basal disease resistance and resistance (R) gene-mediated effector triggered immunity (ETI). Regulates accumulation of the hormone salicylic acid (SA) which is a necessary component of systemic immunity. Involved in responds to bacteria, viruses and oomycetes. References: PMID:11574472, PMID:16040633 Sources: GOC:bhm Also known as: EDS1-PAD4 complex, EDS1-PAD4-SAG101 complex, EDS1-SAG101 complex